{
  "term_label": "smooth muscle cell differentiation",
  "gene_name": "Myocardin",
  "gene_symbol": "MYOCD",
  "term_id": "GO:0051145",
  "gene": "UniProtKB:Q8IZQ8"
}